{
  "term_label": "Unknown biological process",
  "gene_name": "Glycosylated lysosomal membrane protein",
  "term_id": "UNKNOWN:0002",
  "gene_symbol": "GLMP",
  "gene": "UniProtKB:Q8WWB7"
}